{
  "gene_symbol": "PLVAP",
  "term_id": "GO:0002693",
  "gene": "UniProtKB:Q9BX97",
  "term_label": "positive regulation of cellular extravasation",
  "gene_name": "Plasmalemma vesicle-associated protein"
}